{
  "gene_symbol": "WBP11",
  "term_label": "protein phosphatase regulator activity",
  "term_id": "GO:0019888",
  "gene": "UniProtKB:Q9Y2W2",
  "gene_name": "WW domain-binding protein 11"
}